Mcs4 RR-MAPKKK complex [GO:1990315] (cellular component) Relationships: is a type of protein-containing complex [GO:0032991] Note: In S. pombe it consists of Mpr1, Tdh1, Mcs4, Win1, Wis4 and Wis1. Definition: A protein complex that consists of a phospho relay component and a MAPK cascade component. The complex is involved in signaling oxidative stress and osmostress. References: PMID:24255738